mating projection tip [GO:0043332] (cellular component) Sources: GOC:mcc Relationships: is a type of site of polarized growth [GO:0030427]; is a type of cell tip [GO:0051286]; is part of mating projection [GO:0005937] Definition: The apex of the mating projection in unicellular fungi exposed to mating pheromone; site of polarized growth. Also known as: conjugation tube tip, shmoo tip